{
  "gene_symbol": "ESPL1",
  "gene_name": "Separin",
  "term_id": "GO:0005634",
  "term_label": "nucleus",
  "gene": "UniProtKB:Q14674"
}